{
  "term_id": "GO:0061709",
  "gene_name": "Serine_threonine-protein kinase ULK1",
  "term_label": "reticulophagy",
  "gene_symbol": "ULK1",
  "gene": "UniProtKB:O75385"
}